{
  "gene_name": "Nuclear pore complex-interacting protein family member B6",
  "term_label": "Unknown cellular component",
  "gene_symbol": "NPIPB6",
  "term_id": "UNKNOWN:0003",
  "gene": "UniProtKB:E9PJ23"
}